{
  "term_id": "GO:0004823",
  "gene_name": "Leucine--tRNA ligase, mitochondrial",
  "term_label": "leucine-tRNA ligase activity",
  "gene_symbol": "LARS2",
  "gene": "UniProtKB:Q15031"
}